{
  "term_id": "GO:0005737",
  "term_label": "cytoplasm",
  "gene": "UniProtKB:Q6JQN1",
  "gene_symbol": "ACAD10",
  "gene_name": "Acyl-CoA dehydrogenase family member 10"
}